{
  "gene": "UniProtKB:P50993",
  "term_label": "sodium:potassium-exchanging ATPase complex",
  "gene_symbol": "ATP1A2",
  "gene_name": "Sodium_potassium-transporting ATPase subunit alpha-2",
  "term_id": "GO:0005890"
}